{
  "gene": "UniProtKB:Q96LD8",
  "gene_symbol": "SENP8",
  "term_id": "GO:0000338",
  "gene_name": "Sentrin-specific protease 8",
  "term_label": "protein deneddylation"
}